{
  "term_label": "neuronal cell body membrane",
  "term_id": "GO:0032809",
  "gene_symbol": "KCNC1",
  "gene": "UniProtKB:P48547",
  "gene_name": "Potassium voltage-gated channel subfamily C member 1"
}